{
  "gene": "UniProtKB:P55197",
  "term_id": "GO:0005634",
  "term_label": "nucleus",
  "gene_symbol": "MLLT10",
  "gene_name": "Protein AF-10"
}